{
  "gene_symbol": "FOXN2",
  "gene": "UniProtKB:P32314",
  "term_label": "DNA-binding transcription factor activity",
  "term_id": "GO:0003700",
  "gene_name": "Forkhead box protein N2"
}